lactate racemization [GO:0019247] (biological process) Definition: Partial conversion of one lactate enantiomer into another so that the specific optical rotation is decreased, or even reduced to zero, in the resulting mixture. Relationships: is a type of GO:0006089 References: PMID:16166538 Sources: GOC:curators